response to acetylcholine [GO:1905144] (biological process) Definition: Any process that results in a change in state or activity of a cell or an organism (in terms of movement, secretion, enzyme production, gene expression, etc.) as a result of an acetylcholine stimulus. References: PMID:21238497 Sources: GOC:TermGenie, GO_REF:0000071 Relationships: is_a GO:1901698; is_a response to oxygen-containing compound [GO:1901700] Subtypes: cellular response to acetylcholine [GO:1905145]